{
  "term_id": "UNKNOWN:0002",
  "gene_symbol": "EDDM13",
  "gene": "UniProtKB:A0A1B0GTR0",
  "term_label": "Unknown biological process",
  "gene_name": "Epididymal protein 13"
}